alkane transmembrane transporter activity [GO:0015567] (MF) Sources: GOC:ai Definition: Enables the transfer of alkanes from one side of a membrane to the other. Alkanes are saturated aliphatic hydrocarbon compounds. Relationships: is a type of transmembrane transporter activity [GO:0022857]; is part of alkane transport [GO:0015895]